{
  "gene": "UniProtKB:P52741",
  "term_id": "GO:0000122",
  "gene_name": "Zinc finger protein 134",
  "gene_symbol": "ZNF134",
  "term_label": "negative regulation of transcription by RNA polymerase II"
}